{
  "term_label": "calcium ion transmembrane import into cytosol",
  "gene_name": "Transient receptor potential cation channel subfamily A member 1",
  "gene_symbol": "TRPA1",
  "gene": "UniProtKB:O75762",
  "term_id": "GO:0097553"
}